{
  "term_label": "ubiquitin-dependent protein catabolic process",
  "gene_symbol": "UBQLN4",
  "gene": "UniProtKB:Q9NRR5",
  "term_id": "GO:0006511",
  "gene_name": "Ubiquilin-4"
}